{
  "term_id": "GO:0060828",
  "term_label": "regulation of canonical Wnt signaling pathway",
  "gene_name": "Leucine-rich repeat serine_threonine-protein kinase 2",
  "gene": "UniProtKB:Q5S007",
  "gene_symbol": "LRRK2"
}